{
  "term_label": "cytoplasm",
  "gene_symbol": "ETNK1",
  "gene": "UniProtKB:Q9HBU6",
  "gene_name": "Ethanolamine kinase 1",
  "term_id": "GO:0005737"
}